regulation of F-9775B biosynthetic process [GO:1900675] (biological process) Definition: Any process that modulates the frequency, rate or extent of F-9775B biosynthetic process. Sources: GOC:TermGenie, GOC:di Also known as: regulation of F-9775B anabolism, regulation of F-9775B biosynthesis, regulation of F-9775B formation, regulation of F-9775B synthesis Relationships: is a type of GO:1900732; regulates GO:1900614 Subtypes: GO:1900676, positive regulation of F-9775B biosynthetic process [GO:1900677]